{
  "gene_name": "Zinc finger protein 578",
  "gene_symbol": "ZNF578",
  "term_label": "regulation of transcription by RNA polymerase II",
  "term_id": "GO:0006357",
  "gene": "UniProtKB:Q96N58"
}